thioesterase binding [GO:0031996] (molecular function) Sources: GOC:dl Also known as: thiolesterase binding Definition: Binding to a thioesterase. Relationships: is a type of GO:0019899